{
  "term_id": "UNKNOWN:0003",
  "gene": "UniProtKB:P85037",
  "term_label": "Unknown cellular component",
  "gene_name": "Forkhead box protein K1",
  "gene_symbol": "FOXK1"
}